{
  "term_id": "UNKNOWN:0003",
  "gene_name": "Keratin-associated protein 19-1",
  "gene": "UniProtKB:Q8IUB9",
  "gene_symbol": "KRTAP19-1",
  "term_label": "Unknown cellular component"
}